{
  "term_label": "Unknown biological process",
  "term_id": "UNKNOWN:0002",
  "gene": "UniProtKB:Q96ND0",
  "gene_name": "Protein FAM210A",
  "gene_symbol": "FAM210A"
}